polynucleotide adenylyltransferase activator activity [GO:1990749] (molecular function) Definition: Increases the activity of the enzyme polynucleotide adenylyltransferase. References: PMID:19460348 Sources: GOC:kmv Relationships: is a type of enzyme activator activity [GO:0008047]; positively regulates poly(A) RNA polymerase activity [GO:1990817]